{
  "term_id": "UNKNOWN:0001",
  "gene_symbol": "LRRC59",
  "gene": "UniProtKB:Q96AG4",
  "gene_name": "Leucine-rich repeat-containing protein 59",
  "term_label": "Unknown molecular function"
}